{
  "gene": "UniProtKB:Q8TCX1",
  "term_label": "intraciliary retrograde transport",
  "term_id": "GO:0035721",
  "gene_symbol": "DYNC2LI1",
  "gene_name": "Cytoplasmic dynein 2 light intermediate chain 1"
}